{
  "term_id": "GO:0000421",
  "gene_symbol": "GABARAPL2",
  "gene": "UniProtKB:P60520",
  "term_label": "autophagosome membrane",
  "gene_name": "Gamma-aminobutyric acid receptor-associated protein-like 2"
}